fungal-type cell wall (1->3)-alpha-glucan metabolic process [GO:0070599] (biological process) Definition: The chemical reactions and pathways involving (1->3)-alpha-D-glucans, compounds composed of glucose residues linked by (1->3)-alpha-D-glucosidic bonds, found in the walls of ascospores. Relationships: is a type of GO:0070597; is a type of fungal-type cell wall polysaccharide metabolic process [GO:0071966] Also known as: ascospore wall 1,3-alpha-glucan metabolic process, ascospore wall 1,3-alpha-glucan metabolism, ascospore wall alpha-1,3 glucan metabolic process, ascospore wall alpha-1,3 glucan metabolism Subtypes: fungal-type cell wall (1->3)-alpha-glucan biosynthetic process [GO:0070600] Sources: GOC:mah